{
  "gene_symbol": "TRPV3",
  "gene_name": "Transient receptor potential cation channel subfamily V member 3",
  "term_label": "calcium channel activity",
  "term_id": "GO:0005262",
  "gene": "UniProtKB:Q8NET8"
}